{
  "term_label": "cytoplasm",
  "gene_symbol": "THEMIS2",
  "gene_name": "Protein THEMIS2",
  "term_id": "GO:0005737",
  "gene": "UniProtKB:Q5TEJ8"
}